{
  "gene": "UniProtKB:Q16633",
  "term_label": "positive regulation of transcription by RNA polymerase II",
  "gene_name": "POU domain class 2-associating factor 1",
  "term_id": "GO:0045944",
  "gene_symbol": "POU2AF1"
}